{
  "gene_name": "Egl nine homolog 1",
  "term_label": "regulation of neuron apoptotic process",
  "gene": "UniProtKB:Q9GZT9",
  "gene_symbol": "EGLN1",
  "term_id": "GO:0043523"
}